gamma-aminobutyric acid secretion, neurotransmission [GO:0061534] (biological process) Definition: The regulated release of gamma-aminobutyric acid by a cell, in which the gamma-aminobutyric acid acts as a neurotransmitter. Sources: GOC:dph Relationships: is_a neurotransmitter secretion [GO:0007269]; is a type of gamma-aminobutyric acid secretion [GO:0014051]; is part of synaptic transmission, GABAergic [GO:0051932]